{
  "term_label": "Unknown cellular component",
  "gene_name": "Tyrosine-protein phosphatase non-receptor type 20",
  "gene": "UniProtKB:Q4JDL3",
  "gene_symbol": "PTPN20",
  "term_id": "UNKNOWN:0003"
}